{
  "gene": "UniProtKB:Q8WVV4",
  "gene_symbol": "POF1B",
  "term_label": "bicellular tight junction",
  "term_id": "GO:0005923",
  "gene_name": "Protein POF1B"
}